nephron epithelium morphogenesis [GO:0072088] (biological process) Subtypes: nephron tubule morphogenesis [GO:0072078] Definition: The process in which the anatomical structures of the nephron epithelium are generated and organized. The nephron epithelium is a tissue that covers the surface of a nephron. Sources: GOC:mtg_kidney_jan10 Relationships: is a type of morphogenesis of an epithelium [GO:0002009]; is part of nephron epithelium development [GO:0072009]; is part of GO:0072028